{
  "gene_symbol": "OR52I1",
  "term_id": "UNKNOWN:0002",
  "term_label": "Unknown biological process",
  "gene_name": "Olfactory receptor 52I1",
  "gene": "UniProtKB:Q8NGK6"
}